{
  "gene_name": "Syntaxin-4",
  "gene": "UniProtKB:Q12846",
  "term_label": "plasma membrane",
  "term_id": "GO:0005886",
  "gene_symbol": "STX4"
}